ethylbenzene catabolic process [GO:0018915] (biological process) Also known as: ethylbenzene metabolic process, ethylbenzene metabolism Relationships: is a type of benzene-containing compound metabolic process [GO:0042537]; is a type of hydrocarbon catabolic process [GO:0120253] References: PMID:8795196 Subtypes: GO:0010130 Definition: The chemical reactions and pathways resulting in the breakdown of ethylbenzene (phenylethane), a benzene derivative with an ethyl group attached to the ring. It is a colorless liquid with a pungent odor used as a solvent and as a component of automotive and aviation fuels.